regulation of pupariation [GO:0106023] (biological process) Definition: Any process that modulates the onset of pupariation. Relationships: is_a GO:0048580; regulates pupariation [GO:0035073] Subtypes: negative regulation of pupariation [GO:0106024], positive regulation of pupariation [GO:0106025] References: PMID:26510564